{
  "term_label": "axon guidance",
  "term_id": "GO:0007411",
  "gene_name": "Kinesin heavy chain isoform 5C",
  "gene": "UniProtKB:O60282",
  "gene_symbol": "KIF5C"
}